{
  "gene_name": "Insulin-like growth factor-binding protein 5",
  "gene": "UniProtKB:P24593",
  "term_id": "GO:0043567",
  "term_label": "regulation of insulin-like growth factor receptor signaling pathway",
  "gene_symbol": "IGFBP5"
}